dehydro-D-arabinono-1,4-lactone biosynthetic process [GO:0070485] (BP) Also known as: dehydro-D-arabinono-1,4-lactone anabolism, dehydro-D-arabinono-1,4-lactone biosynthesis, dehydro-D-arabinono-1,4-lactone formation, dehydro-D-arabinono-1,4-lactone synthesis Definition: The chemical reactions and pathways resulting in the formation of dehydro-D-arabinono-1,4-lactone, the gamma-lactone (5R)-3,4-dihydroxy-5-(hydroxymethyl)furan-2(5H)-one. Sources: GOC:cjk, GOC:mah Relationships: is a type of GO:1901336